{
  "gene": "UniProtKB:P52294",
  "gene_name": "Importin subunit alpha-5",
  "gene_symbol": "KPNA1",
  "term_id": "GO:0005634",
  "term_label": "nucleus"
}